response to dodecane [GO:1902786] (biological process) Definition: Any process that results in a change in state or activity of a cell or an organism (in terms of movement, secretion, enzyme production, gene expression, etc.) as a result of a dodecane stimulus. References: PMID:23826995 Sources: GOC:TermGenie, GOC:mengo_curators, GO_REF:0000071 Relationships: is_a response to alkane [GO:1902778] Subtypes: cellular response to dodecane [GO:1902787]